{
  "term_label": "mRNA binding",
  "gene": "UniProtKB:O75153",
  "gene_symbol": "CLUH",
  "gene_name": "Clustered mitochondria protein homolog",
  "term_id": "GO:0003729"
}